{
  "term_id": "GO:0003700",
  "term_label": "DNA-binding transcription factor activity",
  "gene": "UniProtKB:Q9BU19",
  "gene_symbol": "ZNF692",
  "gene_name": "Zinc finger protein 692"
}